{
  "gene_name": "Semaphorin-6B",
  "gene": "UniProtKB:Q9H3T3",
  "term_label": "semaphorin-plexin signaling pathway",
  "term_id": "GO:0071526",
  "gene_symbol": "SEMA6B"
}